{
  "term_id": "GO:0004725",
  "term_label": "protein tyrosine phosphatase activity",
  "gene_symbol": "PTP4A2",
  "gene_name": "Protein tyrosine phosphatase type IVA 2",
  "gene": "UniProtKB:Q12974"
}